regulation of T cell antigen processing and presentation [GO:0002625] (biological process) Relationships: is a type of regulation of antigen processing and presentation [GO:0002577]; is_a regulation of T cell mediated immunity [GO:0002709]; regulates T cell antigen processing and presentation [GO:0002457] Definition: Any process that modulates the frequency, rate, or extent of T cell antigen processing and presentation. Subtypes: negative regulation of T cell antigen processing and presentation [GO:0002626], GO:0002627 Sources: GOC:add Also known as: regulation of T lymphocyte antigen processing and presentation, regulation of T-cell antigen processing and presentation, regulation of T-lymphocyte antigen processing and presentation